cephalosporin C biosynthetic process [GO:1901268] (biological process) Relationships: is_a GO:0043646; is a type of carboxylic acid biosynthetic process [GO:0046394]; is a type of cephalosporin C metabolic process [GO:1901266] Sources: GOC:TermGenie, GOC:yaf, UniPathway:UPA00172 Also known as: cephalosporin C anabolism, cephalosporin C biosynthesis, cephalosporin C formation, cephalosporin C synthesis Definition: The chemical reactions and pathways resulting in the formation of cephalosporin C.